pullulan binding [GO:2001067] (molecular function) Relationships: is a type of polysaccharide binding [GO:0030247] Sources: GOC:mengo_curators Definition: Binding to pullulan.